alkylglycerophosphoethanolamine phosphodiesterase activity [GO:0047391] (molecular function) Definition: Catalysis of the reaction: H2O + 1-alkyl-sn-glycero-3-phosphoethanolamine = ethanolamine + 1-alkyl-sn-glycerol 3-phosphate. Sources: EC:3.1.4.39, MetaCyc:3.1.4.39-RXN Also known as: 1-alkyl-sn-glycero-3-phosphoethanolamine ethanolaminehydrolase activity, lysophospholipase D activity Relationships: is a type of GO:0008081